{
  "gene": "UniProtKB:Q9BVC5",
  "gene_symbol": "C2orf49",
  "gene_name": "Ashwin",
  "term_id": "GO:0072669",
  "term_label": "tRNA-splicing ligase complex"
}